{
  "gene": "UniProtKB:P11509",
  "term_id": "GO:0008392",
  "term_label": "arachidonate epoxygenase activity",
  "gene_symbol": "CYP2A6",
  "gene_name": "Cytochrome P450 2A6"
}